{
  "gene_symbol": "TRAV21",
  "gene_name": "T cell receptor alpha variable 21",
  "gene": "UniProtKB:A0A0B4J279",
  "term_id": "UNKNOWN:0001",
  "term_label": "Unknown molecular function"
}